{
  "gene_symbol": "LINC00173",
  "term_id": "UNKNOWN:0002",
  "gene": "UniProtKB:Q6ZV60",
  "gene_name": "Putative uncharacterized protein encoded by LINC00173",
  "term_label": "Unknown biological process"
}